negative regulation of T-helper 1 cell activation [GO:2000518] (biological process) Definition: Any process that stops, prevents or reduces the frequency, rate or extent of T-helper 1 cell activation. Sources: GOC:obol Relationships: is a type of negative regulation of CD4-positive, alpha-beta T cell activation [GO:2000515]; is a type of regulation of T-helper 1 cell activation [GO:2000517]; negatively regulates T-helper 1 cell activation [GO:0035711] Also known as: negative regulation of Th1 cell activation